{
  "term_id": "GO:0007130",
  "gene_symbol": "SYCE3",
  "term_label": "synaptonemal complex assembly",
  "gene": "UniProtKB:A1L190",
  "gene_name": "Synaptonemal complex central element protein 3"
}